{
  "gene_name": "Ras-related protein Rab-7a",
  "term_label": "phagosome-lysosome fusion",
  "gene_symbol": "RAB7A",
  "term_id": "GO:0090385",
  "gene": "UniProtKB:P51149"
}